(+)-2-epi-prezizaene synthase activity [GO:0102201] (molecular function) Relationships: is a type of carbon-oxygen lyase activity, acting on phosphates [GO:0016838] Definition: Catalysis of the reaction: 2-cis,6-trans-farnesyl diphosphate = (+)-2-epi-prezizaene + diphosphoric acid. References: PMID:20175559, PMID:20201526 Sources: GOC:pz